nitrogen catabolite repression of transcription [GO:0090295] (biological process) Definition: A transcription regulation process in which the presence of one nitrogen source leads to a decrease in the frequency, rate, or extent of transcription of specific genes involved in the metabolism of other nitrogen sources. References: PMID:19104072 Sources: GOC:mah, GOC:rb Also known as: negative regulation of transcription by nitrogen catabolites, nitrogen catabolite repression Relationships: is a type of negative regulation of DNA-templated transcription [GO:0045892]; is a type of GO:0061984; is a type of nitrogen catabolite regulation of transcription [GO:0090293] Subtypes: nitrogen catabolite repression of transcription from RNA polymerase II promoter [GO:0001081]